{
  "gene": "UniProtKB:P10916",
  "gene_symbol": "MYL2",
  "gene_name": "Myosin regulatory light chain 2, ventricular_cardiac muscle isoform",
  "term_id": "GO:0060048",
  "term_label": "cardiac muscle contraction"
}